{
  "term_id": "GO:0006357",
  "gene_name": "Zinc finger protein 559",
  "gene_symbol": "ZNF559",
  "gene": "UniProtKB:Q9BR84",
  "term_label": "regulation of transcription by RNA polymerase II"
}